{
  "term_label": "immunoglobulin mediated immune response",
  "term_id": "GO:0016064",
  "gene": "UniProtKB:A0A0B4J2H0",
  "gene_symbol": "IGHV1-69D",
  "gene_name": "Immunoglobulin heavy variable 1-69D"
}